{
  "gene_symbol": "AGXT2",
  "gene": "UniProtKB:Q9BYV1",
  "term_id": "GO:0009436",
  "gene_name": "Alanine--glyoxylate aminotransferase 2, mitochondrial",
  "term_label": "glyoxylate catabolic process"
}